{
  "term_id": "GO:0030350",
  "term_label": "iron-responsive element binding",
  "gene_name": "Iron-responsive element-binding protein 2",
  "gene_symbol": "IREB2",
  "gene": "UniProtKB:P48200"
}